{
  "term_label": "regulation of transcription by RNA polymerase II",
  "gene": "UniProtKB:O15266",
  "gene_symbol": "SHOX",
  "term_id": "GO:0006357",
  "gene_name": "Short stature homeobox protein"
}